{
  "gene": "UniProtKB:Q5SY80",
  "term_id": "GO:0036128",
  "gene_symbol": "CATSPERE",
  "gene_name": "Cation channel sperm-associated auxiliary subunit epsilon",
  "term_label": "CatSper complex"
}